{
  "gene": "UniProtKB:Q7Z5A8",
  "term_id": "GO:1903980",
  "gene_symbol": "TAFA3",
  "gene_name": "Chemokine-like protein TAFA-3",
  "term_label": "positive regulation of microglial cell activation"
}